{
  "gene_name": "Neuropeptide S receptor",
  "term_label": "neuropeptide receptor activity",
  "gene": "UniProtKB:Q6W5P4",
  "gene_symbol": "NPSR1",
  "term_id": "GO:0008188"
}